{
  "term_id": "UNKNOWN:0001",
  "term_label": "Unknown molecular function",
  "gene_symbol": "VPS37C",
  "gene_name": "Vacuolar protein sorting-associated protein 37C",
  "gene": "UniProtKB:A5D8V6"
}